symbiont-mediated suppression of host cell division [GO:0044865] (biological process) Also known as: inhibition by virus of host cell division, negative regulation by virus of host cell division References: PMID:24218612 Relationships: is a type of symbiont-mediated perturbation of host cellular process [GO:0044068] Definition: A process in which a symbiont inhibits or disrupts the normal execution of cell division in the host cell. The host is defined as the larger of the organisms involved in a symbiotic interaction.